{
  "term_id": "GO:0048786",
  "gene_symbol": "PPFIA2",
  "gene": "UniProtKB:O75334",
  "term_label": "presynaptic active zone",
  "gene_name": "Liprin-alpha-2"
}